regulation of protein localization to meiotic spindle pole body [GO:0140433] (biological process) Subtypes: GO:0140434, negative regulation of protein localization to meiotic spindle pole body [GO:0140435] Relationships: is a type of regulation of protein localization to spindle pole body [GO:1902363]; regulates GO:1902441 References: PMID:22438582 Definition: Any process that modulates the frequency, rate or extent of protein localization to a meiotic spindle pole body.